{
  "term_label": "regulation of translation",
  "gene_symbol": "CYFIP1",
  "gene": "UniProtKB:Q7L576",
  "gene_name": "Cytoplasmic FMR1-interacting protein 1",
  "term_id": "GO:0006417"
}